{
  "gene": "UniProtKB:Q96JY6",
  "gene_symbol": "PDLIM2",
  "term_id": "GO:0003779",
  "gene_name": "PDZ and LIM domain protein 2",
  "term_label": "actin binding"
}